{
  "gene_name": "Probable tubulin polyglutamylase TTLL2",
  "gene_symbol": "TTLL2",
  "term_label": "tubulin-glutamic acid ligase activity",
  "gene": "UniProtKB:Q9BWV7",
  "term_id": "GO:0070740"
}